regulation of DNA-templated DNA replication initiation [GO:0030174] (biological process) Relationships: is a type of regulation of DNA-templated DNA replication [GO:0090329]; regulates DNA replication initiation [GO:0006270] Definition: Any process that modulates the frequency, rate or extent of initiation of DNA-dependent DNA replication; the process in which DNA becomes competent to replicate. In eukaryotes, replication competence is established in early G1 and lost during the ensuing S phase. Sources: GOC:mah Subtypes: negative regulation of DNA-templated DNA replication initiation [GO:0032297], positive regulation of DNA-templated DNA replication initiation [GO:0032298], regulation of DNA replication initiation involved in plasmid copy number maintenance [GO:0060909], regulation of mitotic DNA replication initiation [GO:1903466], regulation of initiation of premeiotic DNA replication [GO:1904512] Also known as: regulation of DNA replication initiation, DNA replication licencing, DNA replication licensing, regulation of DNA-dependent DNA replication initiation